{
  "term_label": "protein transport to vacuole involved in ubiquitin-dependent protein catabolic process via the multivesicular body sorting pathway",
  "gene_symbol": "VPS25",
  "gene": "UniProtKB:Q9BRG1",
  "gene_name": "Vacuolar protein-sorting-associated protein 25",
  "term_id": "GO:0043328"
}